maintenance of lens transparency [GO:0036438] (biological process) References: PMID:22095752 Sources: GOC:nhn Definition: A homeostatic process in which the lens is maintained in a highly refractive, transparent state to allow for optimal focusing of light on the retina. Relationships: is_a tissue homeostasis [GO:0001894] Also known as: maintenance of ocular lens transparency, preservation of lens transparency